regulation of neutrophil migration [GO:1902622] (BP) Subtypes: regulation of neutrophil chemotaxis [GO:0090022], negative regulation of neutrophil migration [GO:1902623], GO:1902624, GO:2000389 Relationships: is a type of regulation of leukocyte migration [GO:0002685]; RO_0002211 GO:1990266 Definition: Any process that modulates the frequency, rate or extent of neutrophil migration. References: PMID:1826836 Sources: GOC:TermGenie, GO_REF:0000058